hexose transmembrane transport [GO:0008645] (biological process) Note: Note that this term is not intended for use in annotating lateral movement within membranes. Definition: The process in which hexose is transported across a membrane. Hexoses are aldoses with a chain of six carbon atoms in the molecule. Subtypes: D-allose transmembrane transport [GO:0015754], GO:0015755, fucose transmembrane transport [GO:0015756], GO:0015757, GO:0015761, GO:0015762, GO:0140271, D-glucose transmembrane transport [GO:1904659] Sources: GOC:vw Also known as: high-affinity hexose transport, low-affinity hexose transport, hexose membrane transport, hexose transport Relationships: is a type of GO:0015749